symbiont-mediated suppression of host ethylene-mediated defense response [GO:0052005] (biological process) Also known as: negative regulation by organism of defense-related ethylene-mediated signal transduction pathway in other organism involved in symbiotic interaction, negative regulation by organism of ethylene-mediated defense response of other organism involved in symbiotic interaction, negative regulation by symbiont of defense-related host ethylene-mediated signal transduction pathway, down regulation by symbiont of host ethylene-mediated defense response, down-regulation by symbiont of host ethylene-mediated defense response, downregulation by symbiont of host ethylene-mediated defense response, negative regulation by symbiont of host ethylene-mediated defense response, suppression by organism of host ethylene-mediated defense response, suppression by symbiont of host ethylene-mediated defense response, inhibition by symbiont of host ethylene-mediated defense response Sources: GOC:mtg_pamgo_17jul06 Definition: A process in which a symbiont inhibits or disrupts the normal execution of the ethylene-mediated defense response of the host organism. The host is defined as the larger of the organisms involved in a symbiotic interaction. Relationships: is a type of symbiont-mediated suppression of host defenses [GO:0044414]; is_a GO:0052084